very long-chain fatty acid catabolic process [GO:0042760] (biological process) Note: While there is not universal consensus on the lengths of short-, medium-, long- and very-long-chain fatty acids, the GO uses the definitions in ChEBI (see CHEBI:26666, CHEBI:59554, CHEBI:15904 and CHEBI:27283). Relationships: is a type of very long-chain fatty acid metabolic process [GO:0000038]; is a type of fatty acid catabolic process [GO:0009062] Also known as: very-long-chain fatty acid breakdown, very-long-chain fatty acid catabolic process, very-long-chain fatty acid catabolism, very-long-chain fatty acid degradation Subtypes: very long-chain fatty acid beta-oxidation [GO:0140493] Definition: The chemical reactions and pathways resulting in the breakdown of a very long-chain fatty acid. A very long-chain fatty acid has an aliphatic tail containing more than 22 carbons. References: PMID:7744868